{
  "term_id": "GO:0016529",
  "term_label": "sarcoplasmic reticulum",
  "gene_name": "HCLS1-associated protein X-1",
  "gene": "UniProtKB:O00165",
  "gene_symbol": "HAX1"
}